{
  "gene": "UniProtKB:Q99731",
  "gene_symbol": "CCL19",
  "gene_name": "C-C motif chemokine 19",
  "term_id": "GO:0048020",
  "term_label": "CCR chemokine receptor binding"
}